negative regulation of macrophage cytokine production [GO:0010936] (biological process) Relationships: is a type of negative regulation of cytokine production involved in immune response [GO:0002719]; is a type of GO:0010935; negatively regulates macrophage cytokine production [GO:0010934] Sources: GOC:BHF, GOC:rl Definition: Any process that decreases the rate, frequency or extent of macrophage cytokine production. Macrophage cytokine production is the appearance of a chemokine due to biosynthesis or secretion following a cellular stimulus, resulting in an increase in its intracellular or extracellular levels.